nucleoside diphosphate kinase activity [GO:0004550] (molecular function) Also known as: nucleoside-diphosphate kinase activity, ATP:nucleoside-diphosphate phosphotransferase activity, NDK activity, UDP kinase activity, nucleoside 5'-diphosphate kinase activity, nucleoside 5'-diphosphate phosphotransferase activity, nucleoside diphosphate (UDP) kinase activity, nucleoside diphosphokinase activity, nucleotide phosphate kinase activity, uridine diphosphate kinase activity Relationships: is a type of GO:0016776; is a type of nucleobase-containing compound kinase activity [GO:0019205] Definition: Catalysis of the reaction: ATP + nucleoside diphosphate = ADP + nucleoside triphosphate. Sources: EC:2.7.4.6